{
  "term_id": "UNKNOWN:0001",
  "gene_name": "Tether containing UBX domain for GLUT4",
  "gene_symbol": "ASPSCR1",
  "gene": "UniProtKB:Q9BZE9",
  "term_label": "Unknown molecular function"
}